{
  "term_id": "GO:0005685",
  "gene_symbol": "SNRPC",
  "gene_name": "U1 small nuclear ribonucleoprotein C",
  "term_label": "U1 snRNP",
  "gene": "UniProtKB:P09234"
}